{
  "term_id": "GO:0032481",
  "term_label": "positive regulation of type I interferon production",
  "gene": "UniProtKB:Q86XR7",
  "gene_name": "TIR domain-containing adapter molecule 2",
  "gene_symbol": "TICAM2"
}